8-methylthiopropyl glucosinolate S-oxygenase activity [GO:0080107] (molecular function) References: PMID:18799661 Definition: Catalysis of the reaction: 8-methylthiopropyl-glucosinolate = 8-methylsulfinylpropyl-glucosinolate. Relationships: is a type of GO:0016705